{
  "gene": "UniProtKB:Q969K3",
  "term_id": "GO:0043161",
  "term_label": "proteasome-mediated ubiquitin-dependent protein catabolic process",
  "gene_symbol": "RNF34",
  "gene_name": "E3 ubiquitin-protein ligase RNF34"
}